{
  "gene_symbol": "MDFIC",
  "gene": "UniProtKB:Q9P1T7",
  "gene_name": "MyoD family inhibitor domain-containing protein",
  "term_label": "regulation of Wnt signaling pathway",
  "term_id": "GO:0030111"
}